{
  "term_label": "ferric-chelate reductase (NADPH) activity",
  "gene_name": "Metalloreductase STEAP2",
  "gene_symbol": "STEAP2",
  "term_id": "GO:0052851",
  "gene": "UniProtKB:Q8NFT2"
}